{
  "term_label": "Unknown molecular function",
  "gene": "UniProtKB:A6NCI4",
  "term_id": "UNKNOWN:0001",
  "gene_name": "von Willebrand factor A domain-containing protein 3A",
  "gene_symbol": "VWA3A"
}